{
  "gene_name": "Glutathione S-transferase A5",
  "gene_symbol": "GSTA5",
  "term_id": "GO:0006749",
  "term_label": "glutathione metabolic process",
  "gene": "UniProtKB:Q7RTV2"
}